{
  "gene_name": "Leukotriene B4 receptor 1",
  "term_id": "GO:0001632",
  "term_label": "leukotriene B4 receptor activity",
  "gene_symbol": "LTB4R",
  "gene": "UniProtKB:Q15722"
}